collagen and cuticulin-based cuticle development [GO:0040002] (biological process) Definition: Synthesis and deposition of a collagen and cuticulin-based noncellular, hardened, or membranous secretion from an epithelial sheet. An example of this process is found in Caenorhabditis elegans. Sources: GOC:mtg_sensu Also known as: collagen and cuticulin-based cuticle anabolism, collagen and cuticulin-based cuticle biosynthetic process, collagen and cuticulin-based cuticle formation, collagen and cuticulin-based cuticle synthesis Relationships: is a type of cuticle development [GO:0042335] Subtypes: cuticle development involved in collagen and cuticulin-based cuticle molting cycle [GO:0042338]